carnitine metabolic process, CoA-linked [GO:0019254] (biological process) Sources: GOC:go_curators Relationships: is a type of carnitine metabolic process [GO:0009437] Also known as: carnitine metabolism, CoA-linked Definition: The chemical reactions and pathways involving carnitine, where metabolism is linked to CoA.